{
  "gene_name": "Tripartite motif-containing protein 49",
  "gene_symbol": "TRIM49",
  "term_id": "GO:0005737",
  "term_label": "cytoplasm",
  "gene": "UniProtKB:P0CI25"
}